{
  "term_label": "unfolded protein binding",
  "term_id": "GO:0051082",
  "gene_symbol": "PFDN4",
  "gene": "UniProtKB:Q9NQP4",
  "gene_name": "Prefoldin subunit 4"
}